{
  "gene_symbol": "SLC38A2",
  "gene_name": "Sodium-coupled neutral amino acid symporter 2",
  "gene": "UniProtKB:Q96QD8",
  "term_label": "amino acid transmembrane transport",
  "term_id": "GO:0003333"
}